reelin receptor activity [GO:0038025] (molecular function) References: PMID:12827279, PMID:20223215 Sources: GOC:bf Definition: Combining with the secreted glycoprotein reelin, and transmitting the signal from one side of the membrane to the other to initiate a change in cell activity. Also known as: reeler receptor activity Relationships: is a type of transmembrane signaling receptor activity [GO:0004888]; is part of reelin-mediated signaling pathway [GO:0038026]